{
  "gene_name": "Interleukin-12 subunit beta",
  "term_id": "GO:0005125",
  "term_label": "cytokine activity",
  "gene_symbol": "IL12B",
  "gene": "UniProtKB:P29460"
}